{
  "term_label": "protein processing",
  "gene_symbol": "PRSS41",
  "gene": "UniProtKB:Q7RTY9",
  "term_id": "GO:0016485",
  "gene_name": "Serine protease 41"
}